{
  "gene_symbol": "CARD17P",
  "gene_name": "Putative caspase recruitment domain-containing protein 17P",
  "term_id": "UNKNOWN:0001",
  "gene": "UniProtKB:Q5XLA6",
  "term_label": "Unknown molecular function"
}